{
  "term_id": "GO:0000981",
  "gene": "UniProtKB:O43623",
  "gene_symbol": "SNAI2",
  "term_label": "DNA-binding transcription factor activity, RNA polymerase II-specific",
  "gene_name": "Zinc finger protein SNAI2"
}